{
  "gene": "UniProtKB:Q6ZRF7",
  "gene_symbol": "ZNF818P",
  "term_id": "UNKNOWN:0003",
  "term_label": "Unknown cellular component",
  "gene_name": "Putative zinc finger protein 818"
}